peroxisome membrane class-2 targeting sequence binding [GO:0036106] (molecular function) References: PMID:14709540, PMID:17020786 Sources: GOC:pm Definition: Binding to a class II peroxisomal membrane targeting sequence, any of several sequences of amino acids within a protein that can act as a signal for the localization of the protein into the peroxisome membrane in a PEX19-independent manner. Note: Currently identified mPTSs vary greatly in length, and cannot be distinguished by primary structure analysis, suggesting that the peroxisomal sorting information is not contained within a specific amino acid sequence. There do however appear to be two classes of mPTSs: class 1 mPTSs that are bound by PEX19 and imported in a PEX19-dependent manner, and class 2 mPTSs that are not bound by PEX19 and mediate protein import independently of PEX19. The two classes cannot be defined based on their amino acid sequence. Relationships: is a type of peroxisome membrane targeting sequence binding [GO:0033328] Also known as: class 2 mPTS binding, PEX19-independent mPTS binding